{
  "term_id": "UNKNOWN:0002",
  "term_label": "Unknown biological process",
  "gene": "UniProtKB:Q9Y680",
  "gene_symbol": "FKBP7",
  "gene_name": "Peptidyl-prolyl cis-trans isomerase FKBP7"
}